{
  "gene_symbol": "CRYGD",
  "term_id": "GO:0002088",
  "gene_name": "Gamma-crystallin D",
  "gene": "UniProtKB:P07320",
  "term_label": "lens development in camera-type eye"
}